{
  "gene_name": "Plakophilin-2",
  "term_id": "GO:0002934",
  "term_label": "desmosome organization",
  "gene_symbol": "PKP2",
  "gene": "UniProtKB:Q99959"
}